pinocytosis [GO:0006907] (biological process) Definition: An endocytosis process that results in the uptake of liquid material by cells from their external environment; literally 'cell drinking'. Liquid is enclosed in vesicles, called pinosomes, formed by invagination of the plasma membrane. Sources: ISBN:0198506732 Also known as: clathrin-independent pinocytosis, fluid-phase endocytosis, single-organism pinocytosis Relationships: is a type of GO:0006897 Subtypes: micropinocytosis [GO:0044350], macropinocytosis [GO:0044351] Regulation: regulated by regulation of pinocytosis [GO:0048548]; positively regulated by positive regulation of pinocytosis [GO:0048549]; negatively regulated by GO:0048550